{
  "gene": "UniProtKB:Q6FIF0",
  "gene_symbol": "ZFAND6",
  "term_id": "GO:0031593",
  "gene_name": "AN1-type zinc finger protein 6",
  "term_label": "polyubiquitin modification-dependent protein binding"
}